{
  "gene_name": "Proton-coupled zinc antiporter SLC30A9, mitochondrial",
  "term_id": "GO:0006882",
  "term_label": "intracellular zinc ion homeostasis",
  "gene": "UniProtKB:Q6PML9",
  "gene_symbol": "SLC30A9"
}